DIMBOA glucoside beta-D-glucosidase activity [GO:0102726] (molecular function) Sources: EC:3.2.1.182, GOC:pz Definition: Catalysis of the reaction: (2R)-DIMBOA glucoside + H2O = H+ + DIMBOA + beta-D-glucose. Relationships: is a type of hydrolase activity, hydrolyzing O-glycosyl compounds [GO:0004553]